{
  "term_label": "nucleoplasm",
  "gene": "UniProtKB:Q86SE8",
  "gene_name": "Nucleoplasmin-2",
  "term_id": "GO:0005654",
  "gene_symbol": "NPM2"
}